{
  "gene_name": "Protein S100-A6",
  "gene_symbol": "S100A6",
  "term_label": "Unknown biological process",
  "gene": "UniProtKB:P06703",
  "term_id": "UNKNOWN:0002"
}